{
  "term_label": "cytoplasm",
  "gene_symbol": "EIF2AK4",
  "gene_name": "eIF-2-alpha kinase GCN2",
  "gene": "UniProtKB:Q9P2K8",
  "term_id": "GO:0005737"
}